{
  "gene_symbol": "ALAS1",
  "gene": "UniProtKB:P13196",
  "term_id": "GO:0006783",
  "gene_name": "5-aminolevulinate synthase, non-specific, mitochondrial",
  "term_label": "heme biosynthetic process"
}